{
  "term_id": "GO:0047714",
  "term_label": "galactolipase activity",
  "gene_symbol": "PNLIPRP2",
  "gene": "UniProtKB:P54317",
  "gene_name": "Pancreatic lipase-related protein 2"
}